{
  "gene_symbol": "PTPMT1",
  "term_label": "mitochondrion",
  "gene_name": "Phosphatidylglycerophosphatase and protein-tyrosine phosphatase 1",
  "gene": "UniProtKB:Q8WUK0",
  "term_id": "GO:0005739"
}